morphine biosynthetic process [GO:0097295] (biological process) Relationships: is a type of isoquinoline alkaloid biosynthetic process [GO:0033075]; is a type of morphine metabolic process [GO:0071272] Definition: The chemical reactions and pathways resulting in the formation of morphine, 17-methyl-7,8-didehydro-4,5alpha-epoxymorphinan-3,6alpha-diol. Morphine is a highly potent opiate analgesic psychoactive drug obtained form the opium poppy, Papaver somniferum. Also known as: morphine anabolism, morphine biosynthesis, morphine formation, morphine synthesis References: PMID:19567876 Sources: GOC:yaf